{
  "gene": "UniProtKB:Q8WZ82",
  "gene_name": "Esterase OVCA2",
  "term_label": "nucleus",
  "term_id": "GO:0005634",
  "gene_symbol": "OVCA2"
}